regulation of phosphatidic acid biosynthetic process [GO:1905693] (biological process) Subtypes: negative regulation of phosphatidic acid biosynthetic process [GO:1905694], GO:1905695 References: PMID:23767959 Sources: GOC:PARL, GOC:TermGenie, GOC:bc, GO_REF:0000058 Also known as: regulation of phosphatidic acid anabolism, regulation of phosphatidic acid biosynthesis, regulation of phosphatidic acid formation, regulation of phosphatidic acid synthesis Relationships: is_a regulation of phospholipid biosynthetic process [GO:0071071]; regulates GO:0006654 Definition: Any process that modulates the frequency, rate or extent of phosphatidic acid biosynthetic process.